{
  "gene": "UniProtKB:Q7Z7J9",
  "term_label": "protein kinase binding",
  "gene_name": "Calcium_calmodulin-dependent protein kinase II inhibitor 1",
  "gene_symbol": "CAMK2N1",
  "term_id": "GO:0019901"
}